{
  "gene_symbol": "NABP2",
  "term_label": "response to ionizing radiation",
  "gene": "UniProtKB:Q9BQ15",
  "term_id": "GO:0010212",
  "gene_name": "SOSS complex subunit B1"
}